parasympathetic nervous system development [GO:0048486] (biological process) Definition: The process whose specific outcome is the progression of the parasympathetic nervous system over time, from its formation to the mature structure. The parasympathetic nervous system is one of the two divisions of the vertebrate autonomic nervous system. Parasympathetic nerves emerge cranially as pre ganglionic fibers from oculomotor, facial, glossopharyngeal and vagus and from the sacral region of the spinal cord. Most neurons are cholinergic and responses are mediated by muscarinic receptors. The parasympathetic system innervates, for example: salivary glands, thoracic and abdominal viscera, bladder and genitalia. Sources: FMA:9907, GOC:jid, GOC:sr Relationships: is a type of system development [GO:0048731]; is part of autonomic nervous system development [GO:0048483]